negative regulation of primary miRNA processing [GO:2000635] (biological process) Definition: Any process that stops, prevents or reduces the frequency, rate or extent of primary microRNA processing. Also known as: negative regulation of pri-miRNA processing, negative regulation of primary microRNA processing Sources: GOC:dph, GOC:sl Relationships: is a type of GO:1903799; is a type of regulation of primary miRNA processing [GO:2000634]; negatively regulates primary miRNA processing [GO:0031053]